{
  "term_label": "positive regulation of protein localization to kinetochore",
  "gene_name": "Centromere protein Q",
  "term_id": "GO:1905342",
  "gene": "UniProtKB:Q7L2Z9",
  "gene_symbol": "CENPQ"
}